FHF complex [GO:0070695] (cellular component) Relationships: is a type of GO:0032991; is part of cytoplasm [GO:0005737] Note: Note that the gene/protein name 'APC' should not be confused with the abbreviation for 'anaphase promoting complex'. Definition: A protein complex that is composed of AKTIP/FTS, FAM160A2/p107FHIP, and one or more members of the Hook family of proteins, HOOK1, HOOK2, and HOOK3. The complex is thought to promote vesicle trafficking and/or fusion, and associates with the homotypic vesicular sorting complex (the HOPS complex). References: PMID:18799622 Sources: GOC:ab, GOC:mah